{
  "term_id": "GO:0030425",
  "gene_symbol": "SCGN",
  "gene": "UniProtKB:O76038",
  "term_label": "dendrite",
  "gene_name": "Secretagogin"
}